negative regulation of epithelial cell differentiation involved in kidney development [GO:2000697] (biological process) Definition: Any process that stops, prevents or reduces the frequency, rate or extent of epithelial cell differentiation involved in kidney development. Sources: GOC:mtg_kidney_jan10, GOC:yaf Subtypes: negative regulation of mesenchymal to epithelial transition involved in metanephros morphogenesis [GO:0003340], GO:0072183, negative regulation of mesenchymal to epithelial transition involved in mesonephros morphogenesis [GO:2000085] Relationships: is a type of negative regulation of epithelial cell differentiation [GO:0030857]; is a type of regulation of epithelial cell differentiation involved in kidney development [GO:2000696]; negatively regulates epithelial cell differentiation involved in kidney development [GO:0035850]